neuroendocrine cell differentiation [GO:0061101] (biological process) Subtypes: GO:0003311, thyroid-stimulating hormone-secreting cell differentiation [GO:0060129], neuroendocrine cell differentiation involved in prostate gland acinus development [GO:0060531], lung neuroendocrine cell differentiation [GO:0061100], stomach neuroendocrine cell differentiation [GO:0061102], GO:0061103, GO:0061104 Relationships: is a type of neuron differentiation [GO:0030182]; is a type of neuroepithelial cell differentiation [GO:0060563] Sources: GOC:dph Definition: The process in which a relatively unspecialized cell acquires specialized structural and/or functional features of a neuroendocrine cell. A neuroendocrine cell is a cell that receives input form a neuron which controls the secretion of an endocrine substance.